{
  "gene_symbol": "FBXL15",
  "term_label": "SCF ubiquitin ligase complex",
  "gene": "UniProtKB:Q9H469",
  "term_id": "GO:0019005",
  "gene_name": "F-box_LRR-repeat protein 15"
}